{
  "term_id": "GO:0017025",
  "term_label": "TBP-class protein binding",
  "gene_symbol": "DR1",
  "gene": "UniProtKB:Q01658",
  "gene_name": "Protein Dr1"
}